{
  "gene_symbol": "CDC42EP3",
  "term_label": "positive regulation of pseudopodium assembly",
  "gene_name": "Cdc42 effector protein 3",
  "term_id": "GO:0031274",
  "gene": "UniProtKB:Q9UKI2"
}